{
  "gene_name": "Hyaluronan and proteoglycan link protein 2",
  "gene": "UniProtKB:Q9GZV7",
  "term_label": "perineuronal net",
  "gene_symbol": "HAPLN2",
  "term_id": "GO:0072534"
}